{
  "gene_symbol": "LSMEM2",
  "gene_name": "Leucine-rich single-pass membrane protein 2",
  "term_id": "UNKNOWN:0002",
  "term_label": "Unknown biological process",
  "gene": "UniProtKB:Q8N112"
}